{
  "gene_name": "V-type proton ATPase subunit G 1",
  "gene": "UniProtKB:O75348",
  "gene_symbol": "ATP6V1G1",
  "term_label": "vacuolar proton-transporting V-type ATPase, V1 domain",
  "term_id": "GO:0000221"
}